{
  "gene_symbol": "ADD3",
  "gene": "UniProtKB:Q9UEY8",
  "gene_name": "Gamma-adducin",
  "term_label": "actin filament binding",
  "term_id": "GO:0051015"
}